regulation of growth plate cartilage chondrocyte differentiation [GO:1902733] (biological process) Relationships: is a type of regulation of chondrocyte differentiation involved in endochondral bone morphogenesis [GO:1902738]; regulates growth plate cartilage chondrocyte differentiation [GO:0003418] Definition: Any process that modulates the rate, frequency, or extent of the process in which a chondroblast acquires specialized structural and/or functional features of a chondrocyte that will contribute to the growth of a bone. A chondrocyte is a polymorphic cell that forms cartilage. References: PMID:23212449 Sources: GOC:TermGenie, GO_REF:0000058